negative regulation of heart induction [GO:1901320] (biological process) Relationships: is a type of GO:0051093; is a type of regulation of heart induction [GO:0090381]; RO_0002212 heart induction [GO:0003129] Definition: Any process that stops, prevents or reduces the frequency, rate or extent of heart induction. Sources: GOC:TermGenie Also known as: down regulation of heart induction, down-regulation of heart induction, downregulation of heart induction, inhibition of heart induction